{
  "term_label": "Unknown cellular component",
  "term_id": "UNKNOWN:0003",
  "gene_name": "G antigen 7",
  "gene": "UniProtKB:O76087",
  "gene_symbol": "GAGE7"
}